granum [GO:0009542] (cellular component) Definition: Distinct stack of lamellae seen within chloroplasts. Grana contain the pigments, electron transfer compounds, and enzymes essential to the light-dependent reactions of photosynthesis. Relationships: is a type of cellular anatomical structure [GO:0110165]; is part of chloroplast [GO:0009507] Sources: ISBN:0140514031